{
  "term_label": "Unknown molecular function",
  "gene_symbol": "LINC00474",
  "term_id": "UNKNOWN:0001",
  "gene": "UniProtKB:Q9P2X8",
  "gene_name": "Putative uncharacterized protein encoded by LINC00474"
}